{
  "gene_name": "Pro-neuregulin-1, membrane-bound isoform",
  "gene": "UniProtKB:Q02297",
  "gene_symbol": "NRG1",
  "term_label": "extracellular space",
  "term_id": "GO:0005615"
}